{
  "term_id": "GO:1903259",
  "gene": "UniProtKB:Q9BRP8",
  "gene_name": "Partner of Y14 and mago",
  "term_label": "exon-exon junction complex disassembly",
  "gene_symbol": "PYM1"
}